{
  "term_id": "GO:0042147",
  "gene_symbol": "RAB9A",
  "gene": "UniProtKB:P51151",
  "term_label": "retrograde transport, endosome to Golgi",
  "gene_name": "Ras-related protein Rab-9A"
}